{
  "term_label": "positive regulation of cell population proliferation",
  "gene_symbol": "REG3A",
  "term_id": "GO:0008284",
  "gene_name": "Regenerating islet-derived protein 3-alpha",
  "gene": "UniProtKB:Q06141"
}